{
  "term_id": "UNKNOWN:0003",
  "gene_name": "Myogenin",
  "gene_symbol": "MYOG",
  "term_label": "Unknown cellular component",
  "gene": "UniProtKB:P15173"
}